{
  "term_label": "angiogenesis",
  "gene": "UniProtKB:P23467",
  "gene_symbol": "PTPRB",
  "gene_name": "Receptor-type tyrosine-protein phosphatase beta",
  "term_id": "GO:0001525"
}